sulfur compound binding [GO:1901681] (molecular function) Definition: Binding to a sulfur compound. Subtypes: heparin binding [GO:0008201], penicillin binding [GO:0008658], biotin binding [GO:0009374], thienylcyclohexylpiperidine binding [GO:0016596], thiamine binding [GO:0030975], thiamine pyrophosphate binding [GO:0030976], lipoic acid binding [GO:0031405], GO:0035374, S-nitrosoglutathione binding [GO:0035730], 3-sulfino-L-alanine binding [GO:0036127], thiosulfate binding [GO:0036173], sulfate binding [GO:0043199], GO:0043210, glutathione binding [GO:0043295], lipoamide binding [GO:0043544], GO:0043924, 3'-phosphoadenosine 5'-phosphosulfate binding [GO:0050656], coenzyme A binding [GO:0120225], acyl-CoA binding [GO:0120227], L-cysteine binding [GO:1902485], S-adenosyl-L-methionine binding [GO:1904047], GO:1904399, camalexin binding [GO:2001147] Also known as: sulfur molecular entity binding Relationships: is a type of binding [GO:0005488] Sources: GOC:TermGenie, GOC:pr